{
  "gene_name": "Constitutive coactivator of PPAR-gamma-like protein 1",
  "term_label": "nucleus",
  "gene_symbol": "FAM120A",
  "gene": "UniProtKB:Q9NZB2",
  "term_id": "GO:0005634"
}